positive regulation of osteoclast proliferation [GO:0090290] (biological process) Definition: Any process that increases the rate, frequency, or extent of the multiplication or reproduction of osteoclasts, resulting in the expansion of an osteoclast cell population. Relationships: is a type of GO:0070665; is a type of regulation of osteoclast proliferation [GO:0090289]; positively regulates osteoclast proliferation [GO:0002158] Sources: GOC:tb